{
  "term_label": "regulation of the force of heart contraction",
  "term_id": "GO:0002026",
  "gene_symbol": "GRK2",
  "gene": "UniProtKB:P25098",
  "gene_name": "Beta-adrenergic receptor kinase 1"
}